{
  "gene_name": "ATP-dependent 6-phosphofructokinase, liver type",
  "gene": "UniProtKB:P17858",
  "term_label": "6-phosphofructokinase complex",
  "term_id": "GO:0005945",
  "gene_symbol": "PFKL"
}